positive regulation of mitotic nuclear division [GO:0045840] (biological process) Subtypes: positive regulation of mitotic metaphase/anaphase transition [GO:0045842] Sources: GOC:go_curators Relationships: is a type of regulation of mitotic nuclear division [GO:0007088]; is_a positive regulation of nuclear division [GO:0051785]; is a type of positive regulation of cell cycle process [GO:0090068]; positively regulates mitotic nuclear division [GO:0140014] Definition: Any process that activates or increases the frequency, rate or extent of mitosis. Also known as: positive regulation of mitosis, up regulation of mitosis, up-regulation of mitosis, upregulation of mitosis, activation of mitosis, mitogenic activity, stimulation of mitosis